{
  "term_id": "GO:0060271",
  "gene_symbol": "BBS5",
  "gene": "UniProtKB:Q8N3I7",
  "gene_name": "Bardet-Biedl syndrome 5 protein",
  "term_label": "cilium assembly"
}